exoribonuclease II activity [GO:0008859] (molecular function) Definition: Catalysis of the reaction: RNA + H2O = 5'-phosphomononucleotides. Cleaves RNA in the 3' to 5' direction. Sources: EC:3.1.13.1 Also known as: RNase II activity, 5'-exoribonuclease activity, BN ribonuclease activity, Escherichia coli exo-RNase II, RNase II, ribonuclease II activity, ribonuclease Q Relationships: is a type of GO:0000175